{
  "gene_name": "PRAME family member 6",
  "gene_symbol": "PRAMEF6",
  "term_label": "Cul2-RING ubiquitin ligase complex",
  "gene": "UniProtKB:Q5VXH4",
  "term_id": "GO:0031462"
}